xylanase activity [GO:0097599] (molecular function) Also known as: xylosidase activity Sources: GOC:jh2, ISBN:81-7736-269-0 Definition: Catalysis of the hydrolysis of xylans, homopolysaccharides composed of xylose residues. Subtypes: xylan 1,4-beta-xylosidase activity [GO:0009044], GO:0031176, xylan endo-1,3-beta-xylosidase activity [GO:0033905], xylan 1,3-beta-xylosidase activity [GO:0033914], glucuronoarabinoxylan endo-1,4-beta-xylanase activity [GO:0033940], exoxylanase activity [GO:0097600] Relationships: is a type of hydrolase activity, hydrolyzing O-glycosyl compounds [GO:0004553]